{
  "gene_symbol": "CSN3",
  "gene": "UniProtKB:P07498",
  "term_id": "GO:0005615",
  "term_label": "extracellular space",
  "gene_name": "Kappa-casein"
}